microcin transport [GO:0042884] (biological process) Definition: The directed movement of microcin, a class of glycine-rich, bactericidal peptides (antibiotics) produced by some enteric bacteria, into, out of or within a cell, or between cells, by means of some agent such as a transporter or pore. References: PMID:11292337 Sources: GOC:jl Subtypes: GO:0042885 Relationships: is a type of GO:0042886